{
  "gene_symbol": "HIP1R",
  "gene_name": "Huntingtin-interacting protein 1-related protein",
  "gene": "UniProtKB:O75146",
  "term_label": "actin filament organization",
  "term_id": "GO:0007015"
}